{
  "gene_name": "Protein SOX-15",
  "gene": "UniProtKB:O60248",
  "term_id": "GO:0000122",
  "gene_symbol": "SOX15",
  "term_label": "negative regulation of transcription by RNA polymerase II"
}